{
  "term_id": "GO:0006357",
  "gene": "UniProtKB:Q8TDD2",
  "term_label": "regulation of transcription by RNA polymerase II",
  "gene_symbol": "SP7",
  "gene_name": "Transcription factor Sp7"
}